{
  "term_id": "GO:0017157",
  "gene_symbol": "SEPTIN1",
  "term_label": "regulation of exocytosis",
  "gene_name": "Septin-1",
  "gene": "UniProtKB:Q8WYJ6"
}